{
  "term_id": "UNKNOWN:0001",
  "gene": "UniProtKB:Q96EN9",
  "term_label": "Unknown molecular function",
  "gene_symbol": "REX1BD",
  "gene_name": "Required for excision 1-B domain-containing protein"
}